nucleoside salvage [GO:0043174] (biological process) Relationships: is a type of nucleoside biosynthetic process [GO:0009163]; is a type of metabolic compound salvage [GO:0043094] Sources: GOC:jl Subtypes: purine ribonucleoside salvage [GO:0006166], pyrimidine nucleoside salvage [GO:0043097], GO:0043098 Definition: Any process which produces a nucleotide, a nucleobase linked to either beta-D-ribofuranose (ribonucleoside) or 2-deoxy-beta-D-ribofuranose (a deoxyribonucleotide), from derivatives of it without de novo synthesis.